{
  "gene_name": "Nexilin",
  "gene": "UniProtKB:Q0ZGT2",
  "term_id": "GO:0030424",
  "gene_symbol": "NEXN",
  "term_label": "axon"
}